regulation of mitochondrial rRNA stability [GO:0044529] (biological process) Definition: Any process that modulates the propensity of mitochondrial rRNA molecules to degradation. Includes processes that both stabilize and destabilize mitochondrial rRNAs. Sources: GOC:al, GOC:jl Relationships: is a type of regulation of rRNA stability [GO:0044357]